regulation of cardiac ventricle development [GO:1904412] (biological process) Relationships: is a type of regulation of developmental process [GO:0050793]; regulates cardiac ventricle development [GO:0003231] Definition: Any process that modulates the frequency, rate or extent of cardiac ventricle development. References: PMID:19590510 Sources: GOC:TermGenie, GO_REF:0000058 Subtypes: GO:1904413, positive regulation of cardiac ventricle development [GO:1904414]